{
  "gene_name": "Interleukin-1 receptor antagonist protein",
  "term_id": "GO:0006954",
  "gene_symbol": "IL1RN",
  "term_label": "inflammatory response",
  "gene": "UniProtKB:P18510"
}